generation of mature 5'-end of LSU-rRNA from tricistronic rRNA transcript (SSU-rRNA, 5.8S rRNA, LSU-rRNA) [GO:0000477] (biological process) Relationships: is a type of rRNA 5'-end processing [GO:0000967]; is part of maturation of LSU-rRNA from tricistronic rRNA transcript (SSU-rRNA, 5.8S rRNA, LSU-rRNA) [GO:0000463] Also known as: processing at C1 References: PMID:10690410 Sources: GOC:curators Definition: Cleavage within ITS2 to generate the mature 5'-end of an LSU-rRNA derived from a tricistronic rRNA transcript that contained the Small SubUnit (SSU) rRNA, the 5.8S rRNA, and the Large SubUnit (LSU) rRNA, in that order, from 5' to 3' along the primary transcript.